{
  "gene": "UniProtKB:Q5SY68",
  "term_label": "cytoplasm",
  "gene_name": "Protein S100-A7-like 2",
  "gene_symbol": "S100A7L2",
  "term_id": "GO:0005737"
}